{
  "term_id": "GO:0098655",
  "gene_name": "cGMP-gated cation channel alpha-1",
  "gene_symbol": "CNGA1",
  "gene": "UniProtKB:P29973",
  "term_label": "monoatomic cation transmembrane transport"
}